{
  "gene_symbol": "COL28A1",
  "term_label": "extracellular matrix structural constituent conferring tensile strength",
  "gene": "UniProtKB:Q2UY09",
  "gene_name": "Collagen alpha-1(XXVIII) chain",
  "term_id": "GO:0030020"
}